{
  "gene_name": "72 kDa type IV collagenase",
  "term_label": "metalloendopeptidase activity",
  "gene": "UniProtKB:P08253",
  "gene_symbol": "MMP2",
  "term_id": "GO:0004222"
}